{
  "gene_name": "Oxytocin receptor",
  "gene": "UniProtKB:P30559",
  "term_id": "GO:0045907",
  "gene_symbol": "OXTR",
  "term_label": "positive regulation of vasoconstriction"
}